cell wall polysaccharide biosynthetic process [GO:0070592] (biological process) Definition: The chemical reactions and pathways resulting in the formation of a polysaccharide destined to form part of a cell wall. Sources: GOC:mah Relationships: is a type of polysaccharide biosynthetic process [GO:0000271]; is a type of GO:0010383; is a type of cell wall macromolecule biosynthetic process [GO:0044038] Also known as: cell wall polysaccharide anabolism, cell wall polysaccharide biosynthesis, cell wall polysaccharide synthesis Subtypes: rhamnogalacturonan I biosynthetic process [GO:0010246], cell wall beta-glucan biosynthetic process [GO:0034410], xylan biosynthetic process [GO:0045492], mannan biosynthetic process [GO:0046354], fungal-type cell wall polysaccharide biosynthetic process [GO:0051278], GO:0052325, cell wall (1->3)-alpha-glucan biosynthetic process [GO:0070598]